cyclase activator activity [GO:0010853] (molecular function) Definition: Binds to and increases the activity of an enzyme that catalyzes a ring closure reaction. Subtypes: adenylate cyclase activator activity [GO:0010856], GO:0030250 Relationships: is a type of enzyme activator activity [GO:0008047]; is a type of cyclase regulator activity [GO:0010851]; positively regulates cyclase activity [GO:0009975] Sources: GOC:dph, GOC:tb